{
  "gene_name": "Interleukin-11 receptor subunit alpha",
  "term_id": "GO:0004921",
  "gene_symbol": "IL11RA",
  "gene": "UniProtKB:Q14626",
  "term_label": "interleukin-11 receptor activity"
}